positive regulation of neutrophil aggregation [GO:2000430] (biological process) Sources: GOC:BHF Also known as: positive regulation of neutrocyte aggregation, positive regulation of neutrophil leucocyte aggregation, positive regulation of neutrophilic leukocyte aggregation Definition: Any process that activates or increases the frequency, rate or extent of neutrophil aggregation. Relationships: is a type of positive regulation of leukocyte cell-cell adhesion [GO:1903039]; is_a regulation of neutrophil aggregation [GO:2000428]; positively regulates neutrophil aggregation [GO:0070488]